CD4 receptor binding [GO:0042609] (molecular function) Definition: Binding to a CD4, a receptor found on the surface of T cells, monocytes and macrophages. Relationships: is a type of GO:0005102 Sources: GOC:jl, MSH:D015704